myosin heavy chain kinase activity [GO:0016905] (molecular function) Definition: Catalysis of the reaction: ATP + myosin-heavy-chain = ADP + myosin-heavy-chain phosphate. Sources: EC:2.7.11.7 Also known as: myosin I heavy chain kinase activity, myosin I heavy-chain kinase activity, myosin II heavy chain kinase activity, myosin II heavy-chain kinase activity, ATP:myosin heavy-chain O-phosphotransferase activity, ATP:myosin-heavy-chain O-phosphotransferase activity, MHCK, MIHC kinase activity, STK6, calmodulin-dependent myosin heavy chain kinase activity, myosin heavy chain kinase A activity, myosin heavy-chain kinase activity, myosin-heavy-chain kinase activity Relationships: is a type of calcium/calmodulin-dependent protein kinase activity [GO:0004683]